methylumbelliferyl-acetate deacetylase activity [GO:0047374] (molecular function) Also known as: 4-methylumbelliferyl-acetate acylhydrolase activity, esterase D activity Relationships: is a type of deacetylase activity [GO:0019213]; is a type of carboxylic ester hydrolase activity [GO:0052689] Sources: EC:3.1.1.56, RHEA:12208 Definition: Catalysis of the reaction: 4-methylumbelliferyl acetate + H2O = 4-methylumbelliferone + acetate + H+.